{
  "gene_symbol": "CATSPER2",
  "gene": "UniProtKB:Q96P56",
  "gene_name": "Cation channel sperm-associated protein 2",
  "term_id": "GO:0036128",
  "term_label": "CatSper complex"
}